{
  "term_id": "UNKNOWN:0001",
  "gene_name": "SEC14-like protein 2",
  "gene_symbol": "SEC14L2",
  "gene": "UniProtKB:O76054",
  "term_label": "Unknown molecular function"
}